{
  "gene_name": "Golgin subfamily A member 6C",
  "gene": "UniProtKB:A6NDK9",
  "term_label": "Golgi cis cisterna",
  "gene_symbol": "GOLGA6C",
  "term_id": "GO:0000137"
}